{
  "gene_symbol": "ATF1",
  "gene_name": "Cyclic AMP-dependent transcription factor ATF-1",
  "term_label": "regulation of transcription by RNA polymerase II",
  "term_id": "GO:0006357",
  "gene": "UniProtKB:P18846"
}